{
  "term_label": "chromatin remodeling",
  "term_id": "GO:0006338",
  "gene_name": "Protein-arginine deiminase type-4",
  "gene": "UniProtKB:Q9UM07",
  "gene_symbol": "PADI4"
}